induction of programmed cell death by hormones [GO:0035081] (biological process) Sources: GOC:bf Definition: Any process induced by hormones that directly activates any of the steps required for programmed cell death. Subtypes: induction of programmed cell death by ecdysone [GO:0035078] Relationships: is a type of GO:0012502